{
  "gene_symbol": "MT-ND6",
  "gene": "UniProtKB:P03923",
  "gene_name": "NADH-ubiquinone oxidoreductase chain 6",
  "term_id": "UNKNOWN:0001",
  "term_label": "Unknown molecular function"
}